{
  "term_label": "DNA endonuclease activity",
  "term_id": "GO:0004520",
  "gene_symbol": "BIVM",
  "gene_name": "Basic immunoglobulin-like variable motif-containing protein",
  "gene": "UniProtKB:Q86UB2"
}